{
  "term_id": "GO:0031466",
  "gene_symbol": "RNF7",
  "term_label": "Cul5-RING ubiquitin ligase complex",
  "gene": "UniProtKB:Q9UBF6",
  "gene_name": "RING-box protein 2"
}